{
  "term_id": "GO:0005730",
  "gene_name": "Protein FRG1",
  "gene": "UniProtKB:Q14331",
  "term_label": "nucleolus",
  "gene_symbol": "FRG1"
}